N-acylmannosamine 1-dehydrogenase activity [GO:0050123] (molecular function) Sources: EC:1.1.1.233, RHEA:11540 Also known as: N-acetyl-D-mannosamine dehydrogenase activity, N-acyl-D-mannosamine dehydrogenase activity, N-acyl-D-mannosamine:NAD+ 1-oxidoreductase activity, N-acylmannosamine dehydrogenase activity Definition: Catalysis of the reaction: N-acyl-D-mannosamine + NAD+ = N-acyl-D-mannosaminolactone + H+ + NADH. Relationships: is_a GO:0016616